{
  "gene_name": "Heat shock protein beta-1",
  "gene": "UniProtKB:P04792",
  "gene_symbol": "HSPB1",
  "term_id": "GO:0005737",
  "term_label": "cytoplasm"
}